{
  "gene_symbol": "PAGE4",
  "term_label": "Unknown biological process",
  "gene_name": "P antigen family member 4",
  "gene": "UniProtKB:O60829",
  "term_id": "UNKNOWN:0002"
}